{
  "gene": "UniProtKB:P33121",
  "term_label": "membrane",
  "term_id": "GO:0016020",
  "gene_symbol": "ACSL1",
  "gene_name": "Long-chain-fatty-acid--CoA ligase 1"
}